{
  "term_label": "reticulophagy",
  "gene_name": "Sorting nexin-30",
  "gene": "UniProtKB:Q5VWJ9",
  "term_id": "GO:0061709",
  "gene_symbol": "SNX30"
}